organ or tissue specific immune response [GO:0002251] (biological process) Definition: An immune response taking place in an organ or tissues such as the liver, brain, mucosa, or nervous system tissues. Sources: GOC:jal, GO_REF:0000022 Also known as: immune response in organ or tissue Relationships: is a type of GO:0006955 Subtypes: immune response in brain or nervous system [GO:0002383], hepatic immune response [GO:0002384], GO:0002385